13-hydroxylupinine O-tigloyltransferase activity [GO:0047203] (molecular function) Sources: RHEA:12360 Also known as: (E)-2-methylcrotonoyl-CoA:13-hydroxylupinine O-2-methylcrotonoyltransferase activity, 13-hydroxylupanine acyltransferase activity, tigloyl-CoA:13-hydroxylupanine O-tigloyltransferase activity Relationships: is a type of acyltransferase activity, transferring groups other than amino-acyl groups [GO:0016747] Definition: Catalysis of the reaction: 13-hydroxylupanine + 2-methylcrotonoyl-CoA = 13-(2-methylcrotonoyloxy)lupanine + CoA.